commissural neuron axon guidance [GO:0071679] (biological process) Relationships: is a type of axon guidance [GO:0007411] Sources: GOC:BHF, GOC:mah Definition: The process in which the migration of an axon growth cone of a commissural neuron is directed to its target in the brain in response to a combination of attractive and repulsive cues. Also known as: commissural neuron axon pathfinding